{
  "term_label": "extracellular space",
  "term_id": "GO:0005615",
  "gene": "UniProtKB:P03973",
  "gene_symbol": "SLPI",
  "gene_name": "Antileukoproteinase"
}